negative regulation of alpha-beta T cell differentiation [GO:0046639] (biological process) Also known as: down regulation of alpha-beta T cell differentiation, down-regulation of alpha-beta T cell differentiation, downregulation of alpha-beta T cell differentiation, negative regulation of alpha-beta T lymphocyte differentiation, negative regulation of alpha-beta T-cell differentiation, negative regulation of alpha-beta T-lymphocyte differentiation, inhibition of alpha-beta T cell differentiation, negative regulation of alpha-beta T cell development Note: Note that immunologists typically use the word 'development' to refer to cells of B or T cell lineages undergoing the process that GO describes as 'cell differentiation'. Definition: Any process that stops, prevents, or reduces the frequency, rate or extent of alpha-beta T cell differentiation. Sources: GOC:ai Relationships: is a type of negative regulation of T cell differentiation [GO:0045581]; is a type of GO:0046636; is a type of regulation of alpha-beta T cell differentiation [GO:0046637]; negatively regulates alpha-beta T cell differentiation [GO:0046632] Subtypes: negative regulation of CD4-positive, alpha-beta T cell differentiation [GO:0043371], GO:0043377, negative regulation of NK T cell differentiation [GO:0051137]